ubiquitin-like protein transferase activity [GO:0019787] (molecular function) Subtypes: ubiquitin-protein transferase activity [GO:0004842], FAT10 transferase activity [GO:0019775], GO:0019777, NEDD8 transferase activity [GO:0019788], SUMO transferase activity [GO:0019789], GO:0042294, ISG15 transferase activity [GO:0042296], ubiquitin-like protein conjugating enzyme activity [GO:0061650], GO:0061659, UFM1 transferase activity [GO:0071568], Pup transferase activity [GO:0072496] Definition: Catalysis of the transfer of a ubiquitin-like from one protein to another via the reaction X-ULP + Y = Y-ULP + X, where both X-ULP and Y-ULP are covalent linkages. ULP represents a ubiquitin-like protein. Relationships: is a type of aminoacyltransferase activity [GO:0016755]; is a type of catalytic activity, acting on a protein [GO:0140096] References: PMID:10806345, PMID:10884686 Sources: GOC:mah, GOC:rn Also known as: E2, small conjugating protein transferase activity, small conjugating protein ligase activity, small protein conjugating enzyme activity, ubiquitin-like conjugating enzyme activity, ubiquitin-like-protein ligase activity, E3